subpallium development [GO:0021544] (biological process) References: PMID:12626695 Sources: GOC:cls, GOC:dgh, GOC:dph, GOC:jid, GO_REF:0000021 Relationships: is a type of anatomical structure development [GO:0048856]; is part of telencephalon development [GO:0021537] Definition: The process whose specific outcome is the progression of the subpallium over time, from its formation to the mature structure. The subpallium is the base region of the telencephalon.